{
  "term_label": "Unknown biological process",
  "gene_name": "Reticulocalbin-3",
  "gene": "UniProtKB:Q96D15",
  "gene_symbol": "RCN3",
  "term_id": "UNKNOWN:0002"
}